{
  "gene": "UniProtKB:E5RIL1",
  "gene_name": "Uroplakin-3b-like protein 2",
  "gene_symbol": "UPK3BL2",
  "term_label": "Unknown biological process",
  "term_id": "UNKNOWN:0002"
}